{
  "gene": "UniProtKB:P10323",
  "term_id": "GO:0007340",
  "gene_name": "Acrosin",
  "gene_symbol": "ACR",
  "term_label": "acrosome reaction"
}